{
  "gene_name": "EGF-containing fibulin-like extracellular matrix protein 2",
  "term_id": "UNKNOWN:0001",
  "gene_symbol": "EFEMP2",
  "gene": "UniProtKB:O95967",
  "term_label": "Unknown molecular function"
}